myo-inositol:sodium symporter activity [GO:0005367] (molecular function) Definition: Enables the transfer of a solute or solutes from one side of a membrane to the other according to the reaction: myo-inositol(out) + Na+(out) = myo-inositol(in) + Na+(in). Relationships: is a type of myo-inositol transmembrane transporter activity [GO:0005365]; is a type of solute:sodium symporter activity [GO:0015370] Sources: TC:2.A.21.4.- Also known as: myo-inositol-sodium cotransporter activity